{
  "gene_symbol": "CIPC",
  "gene_name": "CLOCK-interacting pacemaker",
  "term_id": "GO:0005634",
  "term_label": "nucleus",
  "gene": "UniProtKB:Q9C0C6"
}